plasma membrane region [GO:0098590] (CC) Also known as: region of plasma membrane Definition: A membrane that is a (regional) part of the plasma membrane. Subtypes: basal plasma membrane [GO:0009925], basolateral plasma membrane [GO:0016323], apical plasma membrane [GO:0016324], apicolateral plasma membrane [GO:0016327], cell projection membrane [GO:0031253], plasma membrane of cell tip [GO:0031520], plasma membrane-derived thylakoid membrane [GO:0031676], cleavage furrow [GO:0032154], GO:0044853, photoreceptor inner segment membrane [GO:0060342], synaptic membrane [GO:0097060], caveola neck [GO:0099400], cellularization cleavage furrow [GO:0110070], apical plasma membrane urothelial plaque [GO:0120001], hinge region between urothelial plaques of apical plasma membrane [GO:0120003], GO:0120267, periciliary membrane compartment [GO:1990075], sperm head plasma membrane [GO:1990913] Note: Note that this term should not be used for direct manual annotation as it should always be possible to choose a more specific subclass. Sources: GOC:dos Relationships: is a type of GO:0016020; is part of GO:0005886